{
  "gene": "UniProtKB:Q8N9R6",
  "gene_name": "CMT1A duplicated region transcript 4 protein",
  "term_label": "Unknown cellular component",
  "term_id": "UNKNOWN:0003",
  "gene_symbol": "CDRT4"
}